histone H3K14ac reader activity [GO:0140015] (molecular function) References: PMID:30110338 Note: Comment: Note that the residue position corresponds to the canonical human H3 histone (UniProtKB:P84243); this residue is conserved across all eukaryotes. Residue 1 is the first residue following removal of the initiating Methionine (Met). Note that each histone is encoded by multiple genes, and sequences may vary across different genes within an organism. Definition: A histone reader that recognizes a histone H3 acetylated at lysine 14. Also known as: histone H3K14ac modified histone binding Relationships: is a type of histone H3 reader activity [GO:0140006]